{
  "gene": "UniProtKB:Q05586",
  "gene_name": "Glutamate receptor ionotropic, NMDA 1",
  "gene_symbol": "GRIN1",
  "term_label": "neuron projection",
  "term_id": "GO:0043005"
}